{
  "term_id": "GO:0034703",
  "gene": "UniProtKB:Q13507",
  "gene_name": "Short transient receptor potential channel 3",
  "gene_symbol": "TRPC3",
  "term_label": "cation channel complex"
}